{
  "term_id": "UNKNOWN:0001",
  "term_label": "Unknown molecular function",
  "gene": "UniProtKB:Q15041",
  "gene_name": "ADP-ribosylation factor-like protein 6-interacting protein 1",
  "gene_symbol": "ARL6IP1"
}